{
  "gene_name": "Neutrophil defensin 1",
  "gene_symbol": "DEFA1B",
  "term_id": "GO:0051673",
  "gene": "UniProtKB:P59665",
  "term_label": "disruption of plasma membrane integrity in another organism"
}